{
  "term_id": "UNKNOWN:0002",
  "gene_symbol": "NOL7",
  "gene": "UniProtKB:Q9UMY1",
  "term_label": "Unknown biological process",
  "gene_name": "Nucleolar protein 7"
}